{
  "term_label": "Unknown cellular component",
  "term_id": "UNKNOWN:0003",
  "gene_symbol": "SMTN",
  "gene_name": "Smoothelin",
  "gene": "UniProtKB:P53814"
}